{
  "term_label": "diacylglycerol metabolic process",
  "gene_name": "Diacylglycerol kinase eta",
  "term_id": "GO:0046339",
  "gene": "UniProtKB:Q86XP1",
  "gene_symbol": "DGKH"
}